{
  "gene": "UniProtKB:P78563",
  "term_id": "GO:0008251",
  "gene_name": "Double-stranded RNA-specific editase 1",
  "term_label": "tRNA-specific adenosine deaminase activity",
  "gene_symbol": "ADARB1"
}